{
  "term_label": "modulation of chemical synaptic transmission",
  "term_id": "GO:0050804",
  "gene": "UniProtKB:O60260",
  "gene_name": "E3 ubiquitin-protein ligase parkin",
  "gene_symbol": "PRKN"
}